{
  "term_label": "coenzyme A biosynthetic process",
  "gene": "UniProtKB:Q13057",
  "gene_name": "Bifunctional coenzyme A synthase",
  "term_id": "GO:0015937",
  "gene_symbol": "COASY"
}